{
  "term_label": "postsynapse to nucleus signaling pathway",
  "gene_name": "Proline-rich protein 7",
  "gene_symbol": "PRR7",
  "gene": "UniProtKB:Q8TB68",
  "term_id": "GO:0099527"
}